{
  "gene_symbol": "KIFC2",
  "gene": "UniProtKB:Q96AC6",
  "term_id": "GO:0048489",
  "gene_name": "Kinesin-like protein KIFC2",
  "term_label": "synaptic vesicle transport"
}